{
  "term_id": "GO:0006357",
  "gene_symbol": "ZNF256",
  "gene": "UniProtKB:Q9Y2P7",
  "gene_name": "Zinc finger protein 256",
  "term_label": "regulation of transcription by RNA polymerase II"
}